{
  "term_label": "calcium-dependent activation of synaptic vesicle fusion",
  "term_id": "GO:0099502",
  "gene": "UniProtKB:O43581",
  "gene_symbol": "SYT7",
  "gene_name": "Synaptotagmin-7"
}